{
  "term_id": "GO:0048006",
  "gene_name": "T-cell surface glycoprotein CD1a",
  "gene": "UniProtKB:P06126",
  "term_label": "antigen processing and presentation, endogenous lipid antigen via MHC class Ib",
  "gene_symbol": "CD1A"
}